{
  "gene_symbol": "ALDH1L2",
  "gene": "UniProtKB:Q3SY69",
  "term_label": "formyltetrahydrofolate dehydrogenase activity",
  "gene_name": "Mitochondrial 10-formyltetrahydrofolate dehydrogenase",
  "term_id": "GO:0016155"
}